{
  "gene_symbol": "ZNF219",
  "term_label": "regulation of DNA-templated transcription",
  "gene": "UniProtKB:Q9P2Y4",
  "gene_name": "Zinc finger protein 219",
  "term_id": "GO:0006355"
}